olfactory nerve structural organization [GO:0021629] (biological process) Relationships: is a type of cranial nerve structural organization [GO:0021604]; is part of olfactory nerve morphogenesis [GO:0021627] Definition: The process that contributes to the act of creating the structural organization of the oculomotor nerve. This process pertains to the physical shaping of a rudimentary structure. The olfactory nerve is a collection of sensory nerve rootlets that extend down from the olfactory bulb to the olfactory mucosa of the upper parts of the nasal cavity. This nerve conducts odor information to the brainstem. Also known as: olfactory nerve structural organisation, CN I structural organization Sources: GOC:cls, GOC:dgh, GOC:dph, GOC:jid, GO_REF:0000021